regulation of modification of postsynaptic actin cytoskeleton [GO:1905274] (biological process) Definition: Any process that modulates the frequency, rate or extent of modification of postsynaptic actin cytoskeleton. References: PMID:21068295 Sources: GOC:TermGenie, GO_REF:0000058 Also known as: regulation of postsynaptic actin cytoskeleton remodelling Relationships: is a type of GO:0099159; RO_0002211 GO:0098885